{
  "term_id": "GO:0005770",
  "gene_symbol": "AP5M1",
  "term_label": "late endosome",
  "gene_name": "AP-5 complex subunit mu-1",
  "gene": "UniProtKB:Q9H0R1"
}